{
  "gene_name": "Sterile alpha motif domain-containing protein 13",
  "gene": "UniProtKB:Q5VXD3",
  "term_id": "UNKNOWN:0003",
  "gene_symbol": "SAMD13",
  "term_label": "Unknown cellular component"
}